{
  "term_label": "olfactory receptor activity",
  "term_id": "GO:0004984",
  "gene_name": "Olfactory receptor 4K5",
  "gene_symbol": "OR4K5",
  "gene": "UniProtKB:Q8NGD3"
}